{
  "term_label": "MAPK cascade",
  "gene_symbol": "MAP3K14",
  "gene": "UniProtKB:Q99558",
  "term_id": "GO:0000165",
  "gene_name": "Mitogen-activated protein kinase kinase kinase 14"
}